methane biosynthetic process from 3-(methylthio)propionic acid [GO:2001132] (biological process) Regulation: regulated by GO:1900333; negatively regulated by negative regulation of methane biosynthetic process from 3-(methylthio)propionic acid [GO:1900334]; positively regulated by GO:1900335 Sources: GOC:mengo_curators Definition: The chemical reactions and pathways resulting in the formation of a methane from a 3-(methylthio)propionic acid. Relationships: is a type of fatty acid metabolic process [GO:0006631]; is a type of sulfur compound metabolic process [GO:0006790]; is a type of methanogenesis [GO:0015948]